{
  "term_id": "GO:0004252",
  "gene_name": "Proprotein convertase subtilisin_kexin type 5",
  "term_label": "serine-type endopeptidase activity",
  "gene": "UniProtKB:Q92824",
  "gene_symbol": "PCSK5"
}